cytoskeletal rearrangement involved in phagocytosis, engulfment [GO:0060097] (BP) Relationships: is a type of cytoskeleton organization [GO:0007010]; is part of phagocytosis, engulfment [GO:0006911] Definition: The assembly, arrangement, or disassembly of cytoskeletal structures that is involved in the internalization of bacteria, immune complexes and other particulate matter or of an apoptotic cell by phagocytosis. Sources: GOC:dph